regulation of phragmoplast microtubule organization [GO:2000694] (biological process) Sources: GOC:obol Relationships: is a type of regulation of microtubule cytoskeleton organization [GO:0070507]; regulates phragmoplast microtubule organization [GO:0080175] Also known as: regulation of phragmoplast microtubule cytoskeleton organization, regulation of phragmoplast microtubule organisation Definition: Any process that modulates the frequency, rate or extent of phragmoplast microtubule organization.